catechol catabolic process, ortho-cleavage [GO:0019615] (biological process) Relationships: is a type of catechol-containing compound catabolic process [GO:0019614]; is a type of beta-ketoadipate pathway [GO:0042952] References: PMID:7765833 Sources: GOC:jl Also known as: catechol breakdown, ortho-cleavage, catechol degradation, ortho-cleavage Definition: The chemical reactions and pathways resulting in the breakdown of catechol via the ortho-cleavage pathway, in which the catechol aromatic ring is broken between the two carbon atoms bearing hydroxyl groups.